{
  "gene_name": "Rho GTPase-activating protein 33",
  "term_id": "GO:0098978",
  "gene": "UniProtKB:O14559",
  "term_label": "glutamatergic synapse",
  "gene_symbol": "ARHGAP33"
}